{
  "gene_symbol": "NEK5",
  "gene_name": "Serine_threonine-protein kinase Nek5",
  "gene": "UniProtKB:Q6P3R8",
  "term_id": "GO:0004672",
  "term_label": "protein kinase activity"
}